{
  "term_label": "regulation of gene expression",
  "gene_name": "Activity-dependent neuroprotector homeobox protein 2",
  "term_id": "GO:0010468",
  "gene": "UniProtKB:Q6IQ32",
  "gene_symbol": "ADNP2"
}